{
  "gene": "UniProtKB:P40938",
  "term_id": "GO:0006261",
  "gene_symbol": "RFC3",
  "term_label": "DNA-templated DNA replication",
  "gene_name": "Replication factor C subunit 3"
}